epinephrine binding [GO:0051379] (molecular function) Also known as: adrenaline binding Definition: Binding to epinephrine, a hormone produced by the medulla of the adrenal glands that increases heart activity, improves the power and prolongs the action of muscles, and increases the rate and depth of breathing. It is synthesized by the methylation of norepinephrine. Sources: GOC:ai Relationships: is a type of GO:0042562; is a type of cation binding [GO:0043169]; is a type of catecholamine binding [GO:1901338]